antigen processing and presentation of endogenous peptide antigen via MHC class I via ER pathway [GO:0002484] (biological process) Relationships: is a type of GO:0019885 Definition: The process in which an antigen-presenting cell expresses a peptide antigen of endogenous origin on its cell surface in association with an MHC class I protein complex following intracellular transport via an ER pathway. The peptide is typically a fragment of a larger endogenous protein which has been degraded within the cell and becomes associated with the MHC class I molecule in the ER. Class I here refers to classical class I molecules. Subtypes: antigen processing and presentation of endogenous peptide antigen via MHC class I via ER pathway, TAP-dependent [GO:0002485], GO:0002486 Also known as: endogenous peptide antigen processing and presentation via MHC class I via ER pathway References: PMID:14647477, PMID:15771591 Sources: GOC:add, ISBN:0781735149